{
  "gene_symbol": "CASP4",
  "term_id": "GO:0005737",
  "gene": "UniProtKB:P49662",
  "term_label": "cytoplasm",
  "gene_name": "Caspase-4"
}